{
  "gene_name": "Ubiquitin carboxyl-terminal hydrolase 22",
  "term_label": "Unknown cellular component",
  "term_id": "UNKNOWN:0003",
  "gene_symbol": "USP22",
  "gene": "UniProtKB:Q9UPT9"
}